{
  "term_id": "UNKNOWN:0001",
  "term_label": "Unknown molecular function",
  "gene_symbol": "CTXN2",
  "gene_name": "Cortexin-2",
  "gene": "UniProtKB:P0C2S0"
}